{
  "term_id": "GO:0047498",
  "term_label": "calcium-dependent phospholipase A2 activity",
  "gene": "UniProtKB:Q9BZM2",
  "gene_symbol": "PLA2G2F",
  "gene_name": "Group IIF secretory phospholipase A2"
}